negative regulation of tonic skeletal muscle contraction [GO:0014748] (biological process) Sources: GOC:ef, GOC:mtg_muscle Definition: Any process that stops, prevents, or reduces the frequency, rate or extent of tonic skeletal muscle contraction. Relationships: is a type of regulation of tonic skeletal muscle contraction [GO:0014746]; is a type of negative regulation of striated muscle contraction [GO:0045988]; negatively regulates GO:0014720